positive regulation of Wnt signaling pathway, calcium modulating pathway [GO:0045813] (biological process) Also known as: positive regulation of Wnt receptor signaling pathway, calcium modulating pathway, positive regulation of Wnt-activated signaling pathway, calcium modulating pathway, positive regulation of frizzled-2 signaling pathway, positive regulation of frizzled-2 signalling pathway, up regulation of frizzled-2 signaling pathway, up-regulation of frizzled-2 signaling pathway, upregulation of frizzled-2 signaling pathway, activation of frizzled-2 signaling pathway, stimulation of frizzled-2 signaling pathway Definition: Any process that activates or increases the frequency, rate or extent of the series of molecular signals initiated by binding of a Wnt protein to a receptor on the surface of the target cell where activated receptors leads to an increase in intracellular calcium and activation of protein kinase C (PKC). Sources: GOC:go_curators Relationships: is a type of regulation of Wnt signaling pathway, calcium modulating pathway [GO:0008591]; is_a GO:2000052; positively regulates Wnt signaling pathway, calcium modulating pathway [GO:0007223]